undecaprenyl-phosphate mannosyltransferase activity [GO:0047267] (molecular function) Sources: EC:2.4.1.54 Definition: Catalysis of the reaction: GDP-mannose + undecaprenyl phosphate = GDP + D-mannosyl-1-phosphoundecaprenol. Also known as: GDP mannose-undecaprenyl phosphate mannosyltransferase activity, GDP-D-mannose:lipid phosphate transmannosylase activity, GDP-mannose:undecaprenyl-phosphate D-mannosyltransferase activity, guanosine diphosphomannose-undecaprenyl phosphate mannosyltransferase activity Relationships: is a type of GO:0000030 Subtypes: GO:0036426, all-trans-undecaprenyl-phosphate mannosyltransferase activity [GO:0036427]